radial spoke stalk [GO:0001536] (cellular component) Definition: Protein complex forming the elongated portion of the radial spoke between the base which binds to the A-tubule of each microtubule outer doublet and the neck which connects to the spoke head within the ciliary or flagellum axoneme. Relationships: is a type of protein-containing complex [GO:0032991]; is part of radial spoke [GO:0001534] References: PMID:22754630, PMID:34871179 Sources: GOC:hjd, GOC:krc